{
  "gene": "UniProtKB:Q70Z44",
  "gene_symbol": "HTR3D",
  "term_label": "transmembrane transporter complex",
  "term_id": "GO:1902495",
  "gene_name": "5-hydroxytryptamine receptor 3D"
}